(S)-mandelate dehydrogenase activity [GO:0033720] (molecular function) Also known as: (S)-2-hydroxy-2-phenylacetate:acceptor 2-oxidoreductase activity, L(+)-mandelate dehydrogenase activity, MDH Definition: Catalysis of the reaction: (S)-2-hydroxy-2-phenylacetate + acceptor = 2-oxo-2-phenylacetate + reduced acceptor. Relationships: is a type of oxidoreductase activity, acting on CH-OH group of donors [GO:0016614] Sources: EC:1.1.99.31